mesonephric nephron development [GO:0061215] (biological process) Definition: The process whose specific outcome is the progression of a nephron in the mesonephros over time, from its formation to the mature structure. A nephron is the functional unit of the kidney. Sources: GOC:mtg_kidney_jan10 Relationships: is a type of GO:0072006; is part of mesonephros development [GO:0001823]